{
  "gene_name": "Ephrin-A1",
  "gene_symbol": "EFNA1",
  "gene": "UniProtKB:P20827",
  "term_label": "axon guidance",
  "term_id": "GO:0007411"
}